propanoate transmembrane transport [GO:0015730] (biological process) Relationships: is a type of short-chain fatty acid transmembrane transport [GO:0015913] Definition: The directed movement of propionate into, out of or within a cell, or between cells, by means of some agent such as a transporter or pore. Sources: GOC:krc Also known as: propanoate transport, propionate transport